regulation of prostatic bud formation [GO:0060685] (biological process) Subtypes: GO:0060514, negative regulation of prostatic bud formation [GO:0060686] Relationships: is a type of GO:0003156; is a type of GO:0060688; is a type of regulation of morphogenesis of an epithelium [GO:1905330]; is a type of regulation of reproductive process [GO:2000241]; regulates prostatic bud formation [GO:0060513] Definition: Any process that modulates the rate, frequency, or extent of prostatic bud formation, the morphogenetic process in which a region of the fetal urogenital sinus epithelium is specified to become the prostate, resulting in prostate bud outgrowth. Sources: GOC:dph